mesenchymal cell proliferation [GO:0010463] (biological process) Subtypes: mesenchymal cell proliferation involved in prostate gland development [GO:0060781], mesenchymal cell proliferation involved in lung development [GO:0060916], kidney mesenchymal cell proliferation [GO:0072135], condensed mesenchymal cell proliferation [GO:0072137], mesenchymal cell proliferation involved in ureteric bud development [GO:0072138], mesenchymal cell proliferation involved in ureter development [GO:0072198], metanephric cap mesenchymal cell proliferation involved in metanephros development [GO:0090094] Definition: The multiplication or reproduction of cells, resulting in the expansion of a mesenchymal cell population. A mesenchymal cell is a cell that normally gives rise to other cells that are organized as three-dimensional masses, rather than sheets. Relationships: is a type of GO:0008283 Regulation: positively regulated by GO:0002053; regulated by regulation of mesenchymal cell proliferation [GO:0010464]; RO_0002212 by negative regulation of mesenchymal cell proliferation [GO:0072201] Sources: GOC:dph, GOC:tb